specification of metanephric loop of Henle identity [GO:0072296] (biological process) Also known as: specification of metanephric intermediate tubule identity Definition: The process in which the loop of Henle of the metanephric nephron acquires its identity. Relationships: is a type of GO:0072086; is a type of specification of metanephric nephron tubule identity [GO:0072293]; is part of GO:0072236 Sources: GOC:bf, GOC:mtg_kidney_jan10